dopaminergic neuron axon guidance [GO:0036514] (biological process) Definition: The chemotaxis process that directs the migration of an axon growth cone of a dopaminergic neuron to a specific target site in response to a combination of attractive and repulsive cues. References: PMID:21106844, PMID:23517308 Sources: GOC:PARL, GOC:bf Also known as: DA axon guidance, dopaminergic axon guidance, mdDA axon guidance Relationships: is a type of axon guidance [GO:0007411]